detection of bacterium [GO:0016045] (biological process) Definition: The series of events in which a stimulus from a bacterium is received and converted into a molecular signal. Subtypes: detection of symbiotic bacterium [GO:0009604] Relationships: is a type of response to bacterium [GO:0009617]; is_a detection of other organism [GO:0098543] Also known as: detection of bacteria, perception of bacteria, perception of bacterium Sources: GOC:hb